N-vanillate-L-glutamate synthetase activity [GO:0052627] (molecular function) Relationships: is a type of acid-amino acid ligase activity [GO:0016881] Definition: Catalysis of the reaction: vanillate + L-glutamate + ATP = N-vanillate-L-glutamate + AMP + diphosphate + H+. Also known as: vanillate amino acid synthetase activity References: PMID:19189963 Sources: MetaCyc:RXN-10885